{
  "gene_name": "Pleckstrin homology domain-containing family O member 2",
  "gene_symbol": "PLEKHO2",
  "gene": "UniProtKB:Q8TD55",
  "term_id": "UNKNOWN:0003",
  "term_label": "Unknown cellular component"
}